T cell receptor binding [GO:0042608] (molecular function) Definition: Binding to a T cell receptor, the antigen-recognizing receptor on the surface of T cells. Also known as: T lymphocyte receptor binding, T-cell receptor binding, T-lymphocyte receptor binding, TCR binding Sources: GOC:jl Relationships: is a type of signaling receptor binding [GO:0005102]; is a type of protein-containing complex binding [GO:0044877]